{
  "gene_symbol": "PRAM1",
  "term_label": "T cell receptor signaling pathway",
  "term_id": "GO:0050852",
  "gene_name": "PML-RARA-regulated adapter molecule 1",
  "gene": "UniProtKB:Q96QH2"
}